{
  "gene": "UniProtKB:Q5VT28",
  "gene_name": "Protein FAM27A_B_C",
  "gene_symbol": "FAM27C",
  "term_label": "Unknown molecular function",
  "term_id": "UNKNOWN:0001"
}